{
  "gene_name": "Tumor necrosis factor receptor superfamily member 1B",
  "term_id": "GO:0031643",
  "term_label": "positive regulation of myelination",
  "gene": "UniProtKB:P20333",
  "gene_symbol": "TNFRSF1B"
}